positive regulation of lipid metabolic process [GO:0045834] (biological process) Definition: Any process that activates or increases the frequency, rate or extent of the chemical reactions and pathways involving lipids. Sources: GOC:go_curators Relationships: is a type of positive regulation of metabolic process [GO:0009893]; is a type of regulation of lipid metabolic process [GO:0019216]; positively regulates lipid metabolic process [GO:0006629] Subtypes: GO:0045923, positive regulation of steroid metabolic process [GO:0045940], positive regulation of lipid biosynthetic process [GO:0046889], positive regulation of lipid catabolic process [GO:0050996], positive regulation of triglyceride metabolic process [GO:0090208], positive regulation of lipid kinase activity [GO:0090218], positive regulation of phospholipid metabolic process [GO:1903727] Also known as: positive regulation of lipid metabolism, up regulation of lipid metabolic process, up-regulation of lipid metabolic process, upregulation of lipid metabolic process, activation of lipid metabolic process, stimulation of lipid metabolic process